{
  "term_label": "cytoplasm",
  "gene_symbol": "PRDX5",
  "gene_name": "Peroxiredoxin-5, mitochondrial",
  "term_id": "GO:0005737",
  "gene": "UniProtKB:P30044"
}